{
  "term_label": "DNA-binding transcription factor activity",
  "gene": "UniProtKB:P47902",
  "gene_symbol": "CDX1",
  "gene_name": "Homeobox protein CDX-1",
  "term_id": "GO:0003700"
}